glycolysis from storage polysaccharide through glucose-1-phosphate [GO:0093001] (biological process) Relationships: is a type of polysaccharide catabolic process [GO:0000272]; is a type of glycolytic process through glucose-1-phosphate [GO:0061622] Definition: The chemical reactions and pathways resulting in the breakdown of a storage polysaccharide into pyruvate through a glucose-1-phosphate intermediate, with the concomitant production of a small amount of ATP and the reduction of NAD to NADH. Sources: GOC:dph, GOC:glycolysis